{
  "gene": "UniProtKB:O95389",
  "term_id": "GO:0007155",
  "term_label": "cell adhesion",
  "gene_name": "Cellular communication network factor 6",
  "gene_symbol": "CCN6"
}